{
  "term_id": "GO:0042627",
  "gene_symbol": "APOA5",
  "gene_name": "Apolipoprotein A-V",
  "term_label": "chylomicron",
  "gene": "UniProtKB:Q6Q788"
}